symbiont-mediated evasion of host immune response [GO:0042783] (biological process) Definition: A process by which an organism avoids the effects of the host organism's immune response. The host is defined as the larger of the organisms involved in a symbiotic interaction. References: PMID:12439615 Sources: GOC:mb Also known as: active evasion of immune response of other organism involved in symbiotic interaction, active immune evasion, evasion or tolerance of host immune response, evasion of host immune response, immune evasion, active evasion of host immune response, evasion by virus of host immune response, mitigation by virus of host immune response, mitigation of host immune response, mitigation of host immune response by virus, passive evasion of host immune response, passive evasion of immune response of other organism involved in symbiotic interaction, passive immune evasion, suppression by virus of host immune response Relationships: is a type of GO:0052553; is a type of response to host immune response [GO:0052572] Subtypes: antigenic variation [GO:0020033], GO:0052165, symbiont-mediated evasion of host innate immune response [GO:0141043]